{
  "gene_symbol": "DDIT3",
  "gene_name": "DNA damage-inducible transcript 3 protein",
  "term_id": "GO:0006983",
  "gene": "UniProtKB:P35638",
  "term_label": "ER overload response"
}